{
  "gene_symbol": "TWF1",
  "term_label": "actin filament",
  "gene": "UniProtKB:Q12792",
  "term_id": "GO:0005884",
  "gene_name": "Twinfilin-1"
}